positive regulation of response to food [GO:0032097] (biological process) Also known as: up regulation of response to food, up-regulation of response to food, upregulation of response to food, activation of response to food, stimulation of response to food Definition: Any process that activates, maintains, or increases the rate of a response to a food stimulus. Sources: GOC:add Relationships: is a type of GO:0032095; is a type of positive regulation of response to nutrient levels [GO:0032109]; positively regulates GO:0032094 Subtypes: GO:0032100, GO:2000141